{
  "gene_symbol": "CFHR1",
  "gene": "UniProtKB:Q03591",
  "term_label": "complement component C3b binding",
  "gene_name": "Complement factor H-related protein 1",
  "term_id": "GO:0001851"
}